{
  "term_label": "cell surface receptor protein serine/threonine kinase signaling pathway",
  "gene_symbol": "BMP15",
  "gene": "UniProtKB:O95972",
  "gene_name": "Bone morphogenetic protein 15",
  "term_id": "GO:0007178"
}